22alpha-hydroxysteroid 23-monooxygenase activity [GO:0102097] (molecular function) Relationships: is_a GO:0016712 Also known as: (22S)-22-hydroxy-5alpha-campestan-3-one C-23 hydroxylase activity Sources: EC:1.14.14.147 Definition: Catalysis of the reaction: (22S,24R)-22-hydroxy-5alpha-ergostan-3-one + O2 + reduced [NADPH--hemoprotein reductase] = 3-dehydro-6-deoxoteasterone + H+ + H2O + oxidized [NADPH--hemoprotein reductase]. Also converts 3-epi-6-deoxocathasterone to 6-deoxotyphasterol.